{
  "term_label": "plasma membrane",
  "gene": "UniProtKB:Q01726",
  "gene_name": "Melanocyte-stimulating hormone receptor",
  "gene_symbol": "MC1R",
  "term_id": "GO:0005886"
}